{
  "gene_name": "E3 ubiquitin-protein ligase TRIM37",
  "term_label": "ubiquitin protein ligase binding",
  "term_id": "GO:0031625",
  "gene": "UniProtKB:O94972",
  "gene_symbol": "TRIM37"
}